{
  "term_id": "GO:0000981",
  "gene": "UniProtKB:Q7L945",
  "gene_name": "Zinc finger protein 627",
  "gene_symbol": "ZNF627",
  "term_label": "DNA-binding transcription factor activity, RNA polymerase II-specific"
}